{
  "gene": "UniProtKB:P52179",
  "term_label": "sarcomere organization",
  "term_id": "GO:0045214",
  "gene_symbol": "MYOM1",
  "gene_name": "Myomesin-1"
}